{
  "gene": "UniProtKB:O15212",
  "term_label": "prefoldin complex",
  "gene_name": "Prefoldin subunit 6",
  "term_id": "GO:0016272",
  "gene_symbol": "PFDN6"
}